{
  "term_label": "cytosol",
  "gene_name": "Dual specificity protein phosphatase 6",
  "term_id": "GO:0005829",
  "gene": "UniProtKB:Q16828",
  "gene_symbol": "DUSP6"
}